{
  "term_label": "mitochondrial membrane",
  "gene_name": "Small integral membrane protein 30",
  "gene_symbol": "SMIM30",
  "term_id": "GO:0031966",
  "gene": "UniProtKB:A4D0T7"
}